acetylcholine metabolic process [GO:0008291] (biological process) Relationships: is a type of metabolic process [GO:0008152] Also known as: acetylcholine metabolism Subtypes: acetylcholine catabolic process [GO:0006581], GO:0008292 Regulation: regulated by regulation of acetylcholine metabolic process [GO:0060408]; positively regulated by GO:0060409 Sources: GOC:jl, GOC:nln, ISBN:0192800752 Definition: The chemical reactions and pathways involving acetylcholine, the acetic acid ester of the organic base choline. Acetylcholine is a major neurotransmitter and neuromodulator both in the central and peripheral nervous systems. It also acts as a paracrine signal in various non-neural tissues.